positive regulation of pinocytosis [GO:0048549] (biological process) Relationships: is_a positive regulation of endocytosis [GO:0045807]; is a type of GO:0048548; RO_0002213 pinocytosis [GO:0006907] Definition: Any process that activates, maintains or increases the rate of pinocytosis. Pinocytosis is the process in which cells take in liquid material from their external environment; literally 'cell drinking'. Liquid is enclosed in vesicles, formed by invagination of the plasma membrane. These vesicles then move into the cell and pass their contents to endosomes. Sources: GOC:go_curators Also known as: up regulation of pinocytosis, up-regulation of pinocytosis, upregulation of pinocytosis, activation of pinocytosis, stimulation of pinocytosis Subtypes: GO:1905303